{
  "gene_name": "Cytoplasmic polyadenylation element-binding protein 2",
  "term_id": "GO:0003730",
  "gene": "UniProtKB:Q7Z5Q1",
  "term_label": "mRNA 3'-UTR binding",
  "gene_symbol": "CPEB2"
}